antiviral innate immune response [GO:0140374] (BP) Relationships: is a type of innate immune response [GO:0045087]; is a type of defense response to virus [GO:0051607] References: PMID:31006531 Definition: A defense response against viruses mediated through an innate immune response. An innate immune response is mediated by germline encoded components that directly recognize components of potential pathogens.